{
  "gene_name": "RING finger protein 175",
  "gene": "UniProtKB:Q8N4F7",
  "term_label": "Golgi membrane",
  "gene_symbol": "RNF175",
  "term_id": "GO:0000139"
}